{
  "gene": "UniProtKB:Q9NWB1",
  "gene_symbol": "RBFOX1",
  "term_label": "regulation of alternative mRNA splicing, via spliceosome",
  "gene_name": "RNA binding protein fox-1 homolog 1",
  "term_id": "GO:0000381"
}